{
  "term_label": "ubiquitin protein ligase activity",
  "gene_symbol": "RNF167",
  "gene_name": "E3 ubiquitin-protein ligase RNF167",
  "term_id": "GO:0061630",
  "gene": "UniProtKB:Q9H6Y7"
}